{
  "gene_symbol": "TSLP",
  "term_label": "extracellular region",
  "gene": "UniProtKB:Q969D9",
  "gene_name": "Thymic stromal lymphopoietin",
  "term_id": "GO:0005576"
}